{
  "gene_name": "Hypermethylated in cancer 2 protein",
  "gene_symbol": "HIC2",
  "term_label": "nucleoplasm",
  "term_id": "GO:0005654",
  "gene": "UniProtKB:Q96JB3"
}